positive regulation of termination of DNA-templated transcription [GO:0060566] (biological process) Definition: Any process that increases the rate, frequency or extent of DNA-templated transcription termination, the process in which transcription is completed; the formation of phosphodiester bonds ceases, the RNA-DNA hybrid dissociates, and RNA polymerase releases the DNA. Also known as: positive regulation of DNA-dependent transcription, termination, positive regulation of DNA-templated transcription, termination, positive regulation of termination of DNA-dependent transcription, positive regulation of transcription termination, DNA-dependent Sources: GOC:dph, GOC:tb, GOC:txnOH Subtypes: transcriptional attenuation [GO:0031555], positive regulation of termination of RNA polymerase II transcription [GO:1904595], positive regulation of termination of RNA polymerase I transcription [GO:2000732] Relationships: is a type of regulation of termination of DNA-templated transcription [GO:0031554]; is a type of positive regulation of protein-containing complex disassembly [GO:0043243]; is a type of positive regulation of DNA-templated transcription [GO:0045893]; positively regulates DNA-templated transcription termination [GO:0006353]